{
  "gene": "UniProtKB:P35080",
  "term_id": "GO:0030833",
  "term_label": "regulation of actin filament polymerization",
  "gene_symbol": "PFN2",
  "gene_name": "Profilin-2"
}